{
  "term_label": "central nervous system development",
  "gene_name": "Versican core protein",
  "gene_symbol": "VCAN",
  "term_id": "GO:0007417",
  "gene": "UniProtKB:P13611"
}